regulation of white fat cell proliferation [GO:0070350] (biological process) Subtypes: negative regulation of white fat cell proliferation [GO:0070351], positive regulation of white fat cell proliferation [GO:0070352] Sources: GOC:mah, GOC:sl Also known as: regulation of white adipocyte proliferation, regulation of white adipose cell proliferation Definition: Any process that modulates the frequency, rate or extent of white fat cell proliferation. Relationships: is a type of GO:0070344; regulates white fat cell proliferation [GO:0070343]